{
  "gene": "UniProtKB:O14786",
  "term_label": "positive regulation of endothelial cell migration",
  "term_id": "GO:0010595",
  "gene_name": "Neuropilin-1",
  "gene_symbol": "NRP1"
}